{
  "gene_symbol": "PCDHGA4",
  "term_id": "GO:0007155",
  "gene": "UniProtKB:Q9Y5G9",
  "gene_name": "Protocadherin gamma-A4",
  "term_label": "cell adhesion"
}